{
  "gene_symbol": "TPR",
  "gene_name": "Nucleoprotein TPR",
  "term_label": "structural constituent of nuclear pore",
  "term_id": "GO:0017056",
  "gene": "UniProtKB:P12270"
}